{
  "gene_name": "Glutamate receptor ionotropic, kainate 1",
  "gene_symbol": "GRIK1",
  "gene": "UniProtKB:P39086",
  "term_label": "transmitter-gated monoatomic ion channel activity involved in regulation of postsynaptic membrane potential",
  "term_id": "GO:1904315"
}